nucleoside:sodium symporter activity [GO:0005415] (molecular function) Also known as: nucleoside-sodium cotransporter activity, sodium-dependent nucleoside transporter activity Sources: GOC:ai Subtypes: pyrimidine- and adenosine-specific:sodium symporter activity [GO:0015389] Relationships: is a type of GO:0005337; is a type of solute:sodium symporter activity [GO:0015370] Definition: Enables the transfer of a solute or solutes from one side of a membrane to the other according to the reaction: nucleoside(out) + Na+(out) = nucleoside(in) + Na+(in).